{
  "term_label": "Unknown cellular component",
  "gene": "UniProtKB:Q9H3R2",
  "gene_symbol": "MUC13",
  "term_id": "UNKNOWN:0003",
  "gene_name": "Mucin-13"
}